piccolo histone acetyltransferase complex [GO:0032777] (cellular component) Definition: A heterotrimeric H4/H2A histone acetyltransferase complex with a substrate preference of chromatin over free histones. It contains a subset of the proteins found in the larger NuA4 histone acetyltransferase complex; for example, the S. cerevisiae complex contains Esa1p, Yng2p, and Epl1p. Relationships: is a type of protein-containing complex [GO:0032991] Subtypes: SAS acetyltransferase complex [GO:0033255] References: PMID:12782659, PMID:15964809 Sources: GOC:rb